{
  "gene_symbol": "SMIM27",
  "gene_name": "Small integral membrane protein 27",
  "term_id": "UNKNOWN:0002",
  "term_label": "Unknown biological process",
  "gene": "UniProtKB:A0A1B0GUW7"
}